laminin-10 complex [GO:0043259] (cellular component) References: PMID:10842354 Sources: GOC:jl Also known as: laminin-511 complex Definition: A laminin complex composed of alpha5, beta1 and gamma1 polypeptide chains. Relationships: is a type of laminin complex [GO:0043256]